{
  "gene_symbol": "PLCB4",
  "gene": "UniProtKB:Q15147",
  "term_id": "GO:0046488",
  "term_label": "phosphatidylinositol metabolic process",
  "gene_name": "1-phosphatidylinositol 4,5-bisphosphate phosphodiesterase beta-4"
}